brassinosteroid binding [GO:0090411] (molecular function) Definition: Binding to a brassinosteroid. Sources: GOC:tb Relationships: is a type of GO:0005496